positive regulation of fibroblast proliferation [GO:0048146] (biological process) Relationships: is a type of GO:0008284; is a type of GO:0048145; positively regulates fibroblast proliferation [GO:0048144] Also known as: up regulation of fibroblast proliferation, up-regulation of fibroblast proliferation, upregulation of fibroblast proliferation, activation of fibroblast proliferation, stimulation of fibroblast proliferation Subtypes: positive regulation of hepatic stellate cell proliferation [GO:1904899], positive regulation of pancreatic stellate cell proliferation [GO:2000231] Sources: GOC:jid Definition: Any process that activates or increases the frequency, rate or extent of multiplication or reproduction of fibroblast cells.